{
  "gene_symbol": "ZNF511",
  "term_id": "UNKNOWN:0001",
  "gene_name": "Zinc finger protein 511",
  "gene": "UniProtKB:Q8NB15",
  "term_label": "Unknown molecular function"
}